{
  "gene_symbol": "SNX13",
  "term_id": "GO:0035091",
  "term_label": "phosphatidylinositol binding",
  "gene": "UniProtKB:Q9Y5W8",
  "gene_name": "Sorting nexin-13"
}